external side of cell outer membrane [GO:0031240] (cellular component) Subtypes: GO:0098568 Sources: GOC:mlg, GOC:mtg_sensu Definition: The side of the outer membrane that is opposite to the side that faces the periplasm of the cell. Relationships: is a type of side of membrane [GO:0098552]; BFO_0000050 cell outer membrane [GO:0009279] Also known as: external leaflet of cell outer membrane, external side of outer membrane Note: In GO, 'external side' still refers to part of the membrane and does not refer to components beyond (outside of) the membrane.